{
  "gene": "UniProtKB:Q99687",
  "term_id": "GO:0009880",
  "gene_name": "Homeobox protein Meis3",
  "term_label": "embryonic pattern specification",
  "gene_symbol": "MEIS3"
}